{
  "gene_symbol": "WNT11",
  "gene_name": "Protein Wnt-11",
  "gene": "UniProtKB:O96014",
  "term_label": "frizzled binding",
  "term_id": "GO:0005109"
}